{
  "gene_name": "Calcyphosin-like protein",
  "gene_symbol": "CAPSL",
  "term_id": "UNKNOWN:0003",
  "gene": "UniProtKB:Q8WWF8",
  "term_label": "Unknown cellular component"
}